{
  "gene": "UniProtKB:Q8NG78",
  "term_label": "olfactory receptor activity",
  "gene_symbol": "OR8G5",
  "term_id": "GO:0004984",
  "gene_name": "Olfactory receptor 8G5"
}